clathrin coat assembly involved in endocytosis [GO:0099049] (biological process) Definition: The process that results in the assembly of clathrin triskelia into a clathrin cage during endocytosis. Clathrin is recruited to the plasma membrane via interaction with scaffolding proteins that bridge between clathtin and cell surface receptors. Clathrin coat formation is concomittant with coated pit formation leading to endocytic vesicle formation. Relationships: is a type of clathrin coat assembly [GO:0048268]; is part of clathrin-dependent endocytosis [GO:0072583] References: PMID:21779028